{
  "term_label": "chromatin DNA binding",
  "gene_symbol": "WBP2NL",
  "gene_name": "Postacrosomal sheath WW domain-binding protein",
  "term_id": "GO:0031490",
  "gene": "UniProtKB:Q6ICG8"
}